{
  "gene_symbol": "SMYD1",
  "gene": "UniProtKB:Q8NB12",
  "term_id": "GO:0005634",
  "gene_name": "Histone-lysine N-methyltransferase SMYD1",
  "term_label": "nucleus"
}